aecium development [GO:0075267] (biological process) Definition: The process in which a cup-like structure containing chains of aeciospores is formed. This is characteristic of the rust fungus and typically, the first dikaryotic spores (aeciospores) are produced in the aecium. Sources: GOC:pamgo_curators Relationships: is a type of GO:0030582 Regulation: regulated by GO:0075268; positively regulated by positive regulation of aecium development [GO:0075269]; negatively regulated by negative regulation of aecium development [GO:0075270]